{
  "gene_name": "Calcium-binding protein 2",
  "gene": "UniProtKB:Q9NPB3",
  "term_id": "GO:0007605",
  "term_label": "sensory perception of sound",
  "gene_symbol": "CABP2"
}